{
  "gene_name": "UDP-glucuronosyltransferase 1A4",
  "term_id": "GO:0016125",
  "term_label": "sterol metabolic process",
  "gene_symbol": "UGT1A4",
  "gene": "UniProtKB:P22310"
}